positive regulation of hematopoietic stem cell migration [GO:2000473] (biological process) Definition: Any process that activates or increases the frequency, rate or extent of hematopoietic stem cell migration. Also known as: positive regulation of hemopoietic stem cell migration Relationships: is a type of positive regulation of cell migration [GO:0030335]; is a type of GO:2000471; positively regulates hematopoietic stem cell migration [GO:0035701] Sources: GOC:obol